{
  "gene": "UniProtKB:Q96G03",
  "term_id": "GO:0006166",
  "gene_name": "Phosphopentomutase",
  "term_label": "purine ribonucleoside salvage",
  "gene_symbol": "PGM2"
}